DNA damage checkpoint signaling [GO:0000077] (biological process) Regulation: regulated by GO:2000001; negatively regulated by negative regulation of DNA damage checkpoint [GO:2000002]; positively regulated by positive regulation of DNA damage checkpoint [GO:2000003] Sources: GOC:mah Definition: A signal transduction process that contributes to a DNA damage checkpoint. Also known as: DNA damage checkpoint, signal transduction involved in DNA damage checkpoint, DNA damage response, signal transduction resulting in cell cycle arrest Relationships: is a type of DNA integrity checkpoint signaling [GO:0031570]; is a type of signal transduction in response to DNA damage [GO:0042770] Subtypes: GO:0044773